glideosome [GO:0160055] (cellular component) Definition: A protein complex composed of at least GAP45 (gliding-associated protein), GAP50 and myosin heavy and light chains. Anchored via GAP50 to the inner membrane complex of motile and invasive forms of apicomplexan parasites and regulates parasite gliding motility and invasion of host cells. Relationships: is a type of GO:0032991 References: PMID:12139608, PMID:15123738, PMID:19577950